{
  "term_label": "nucleus",
  "term_id": "GO:0005634",
  "gene_name": "Histone-lysine N-methyltransferase KMT5B",
  "gene_symbol": "KMT5B",
  "gene": "UniProtKB:Q4FZB7"
}